ion channel inhibitor activity [GO:0008200] (molecular function) Relationships: is a type of GO:0016248; is a type of ion channel regulator activity [GO:0099106]; has part transmembrane transporter binding [GO:0044325]; negatively regulates GO:0005216 Subtypes: GO:0019855, chloride channel inhibitor activity [GO:0019869], potassium channel inhibitor activity [GO:0019870], sodium channel inhibitor activity [GO:0019871] Sources: GOC:mah Definition: Binds to and stops, prevents, or reduces the activity of an ion channel.